{
  "gene_name": "Synaptogyrin-3",
  "term_id": "UNKNOWN:0001",
  "gene": "UniProtKB:O43761",
  "term_label": "Unknown molecular function",
  "gene_symbol": "SYNGR3"
}